{
  "term_id": "GO:0005615",
  "gene_name": "Chemokine-like protein TAFA-4",
  "term_label": "extracellular space",
  "gene": "UniProtKB:Q96LR4",
  "gene_symbol": "TAFA4"
}